granulocyte colony-stimulating factor production [GO:0071611] (biological process) Sources: GOC:add, GOC:rv Also known as: CSF3 production, G-CSF production, colony stimulating factor 3 (granulocyte) production, filgrastim production, granulocyte colony stimulating factor production, lenograstim production, pluripoietin production Relationships: is a type of cytokine production [GO:0001816] Regulation: regulated by regulation of granulocyte colony-stimulating factor production [GO:0071655]; negatively regulated by negative regulation of granulocyte colony-stimulating factor production [GO:0071656]; positively regulated by GO:0071657 Definition: The appearance of granulocyte colony-stimulating factor due to biosynthesis or secretion following a cellular stimulus, resulting in an increase in its intracellular or extracellular levels.